telomere assembly [GO:0032202] (biological process) References: PMID:11902675, PMID:8622671 Sources: GOC:mah, GOC:ns Subtypes: telomere formation via telomerase [GO:0032203] Relationships: is a type of cellular component assembly [GO:0022607]; is a type of telomere organization [GO:0032200] Also known as: telomere formation Definition: A cellular process that results in the aggregation, arrangement and bonding together of a set of components to form a telomere at a non-telomeric double-stranded DNA end. A telomere is a terminal region of a linear chromosome that includes telomeric DNA repeats and associated proteins.